negative regulation of nuclear mRNA surveillance of meiosis-specific transcripts [GO:0120271] (biological process) Also known as: negative regulation of nuclear-transcribed mRNA catabolic process, meiosis-specific transcripts References: PMID:24920274 Sources: GOC:krc Relationships: is a type of regulation of nuclear mRNA surveillance of meiosis-specific transcripts [GO:0120270]; is a type of negative regulation of mRNA catabolic process [GO:1902373]; negatively regulates nuclear mRNA surveillance of meiosis-specific transcripts [GO:0033621] Definition: Any process that stops, prevents or reduces the frequency, rate or extent of selective degradation of meiosis-specific nuclear transcribed transcripts during vegetative growth, by a mechanism that requires determinant of selective removal (DSR) sequences in the targeted mRNAs and involves a YTH family protein.